{
  "gene": "UniProtKB:Q8TCY5",
  "gene_symbol": "MRAP",
  "term_label": "signaling receptor regulator activity",
  "gene_name": "Melanocortin-2 receptor accessory protein",
  "term_id": "GO:0030545"
}